regulation of cleistothecium development [GO:0070796] (biological process) Relationships: is a type of regulation of sporocarp development involved in sexual reproduction [GO:1902058]; regulates cleistothecium development [GO:0070791] Sources: GOC:mah Definition: Any process that modulates the frequency, rate or extent of cleistothecium development, a process that leads to the formation of a cleistothecium. The cleistothecium is a closed sexual fruiting body that contains ascospores in linear asci, characteristic of some filamentous Ascomycete fungi such as members of the genera Aspergillus and Emericella. Subtypes: GO:0070797, positive regulation of cleistothecium development [GO:0070798]